{
  "term_id": "GO:0005737",
  "term_label": "cytoplasm",
  "gene_symbol": "LGALS3",
  "gene": "UniProtKB:P17931",
  "gene_name": "Galectin-3"
}